{
  "gene": "UniProtKB:P49683",
  "term_label": "neuropeptide receptor activity",
  "term_id": "GO:0008188",
  "gene_name": "Prolactin-releasing peptide receptor",
  "gene_symbol": "PRLHR"
}